kinase inhibitor activity [GO:0019210] (molecular function) Subtypes: protein kinase inhibitor activity [GO:0004860] Sources: GOC:mah Definition: Binds to and stops, prevents or reduces the activity of a kinase. Relationships: is a type of GO:0004857; is a type of kinase regulator activity [GO:0019207]; negatively regulates kinase activity [GO:0016301]